{
  "term_label": "regulation of transcription by RNA polymerase II",
  "gene_symbol": "ZNF266",
  "gene": "UniProtKB:Q14584",
  "term_id": "GO:0006357",
  "gene_name": "Zinc finger protein 266"
}